{
  "gene_name": "Protocadherin gamma-A3",
  "gene_symbol": "PCDHGA3",
  "term_label": "cell adhesion molecule binding",
  "term_id": "GO:0050839",
  "gene": "UniProtKB:Q9Y5H0"
}